{
  "gene_symbol": "SYP",
  "term_label": "synaptic vesicle membrane",
  "gene": "UniProtKB:P08247",
  "gene_name": "Synaptophysin",
  "term_id": "GO:0030672"
}